{
  "term_id": "GO:0042420",
  "gene_symbol": "MOXD1",
  "gene_name": "DBH-like monooxygenase protein 1",
  "gene": "UniProtKB:Q6UVY6",
  "term_label": "dopamine catabolic process"
}